{
  "term_id": "GO:0050796",
  "gene": "UniProtKB:P49286",
  "gene_symbol": "MTNR1B",
  "gene_name": "Melatonin receptor type 1B",
  "term_label": "regulation of insulin secretion"
}